negative regulation of CD4-positive, CD25-positive, alpha-beta regulatory T cell differentiation [GO:0032830] (biological process) Definition: Any process that stops, prevents, or reduces the frequency, rate or extent of differentiation of CD4-positive, CD25-positive, alpha-beta regulatory T cells. Note: Note that immunologists typically use the word 'development' to refer to cells of B or T cell lineages undergoing the process that GO describes as 'cell differentiation'. Sources: GOC:mah Relationships: is a type of regulation of CD4-positive, CD25-positive, alpha-beta regulatory T cell differentiation [GO:0032829]; is a type of GO:0043371; is a type of negative regulation of regulatory T cell differentiation [GO:0045590]; negatively regulates CD4-positive, CD25-positive, alpha-beta regulatory T cell differentiation [GO:0002361] Also known as: down regulation of CD4-positive, CD25-positive, alpha-beta regulatory T cell differentiation, down-regulation of CD4-positive, CD25-positive, alpha-beta regulatory T cell differentiation, downregulation of CD4-positive, CD25-positive, alpha-beta regulatory T cell differentiation, negative regulation of CD4-positive, CD25-positive, alpha-beta regulatory T lymphocyte differentiation, negative regulation of CD4-positive, CD25-positive, alpha-beta regulatory T-cell differentiation, negative regulation of CD4-positive, CD25-positive, alpha-beta regulatory T-lymphocyte differentiation, inhibition of CD4-positive, CD25-positive, alpha-beta regulatory T cell differentiation, negative regulation of CD4-positive, CD25-positive, alpha-beta regulatory T cell development Subtypes: negative regulation of CD4-positive, CD25-positive, alpha-beta regulatory T cell differentiation involved in immune response [GO:0032833]